{
  "gene_name": "Akirin-2",
  "term_id": "GO:0003712",
  "term_label": "transcription coregulator activity",
  "gene": "UniProtKB:Q53H80",
  "gene_symbol": "AKIRIN2"
}